{
  "gene_name": "Immunoglobulin heavy variable 3_OR15-7 (pseudogene) (Fragment)",
  "term_label": "immunoglobulin mediated immune response",
  "gene": "UniProtKB:A0A075B7D8",
  "term_id": "GO:0016064",
  "gene_symbol": "IGHV3OR15-7"
}